{
  "term_label": "ribosome binding",
  "gene_name": "Death-associated protein-like 1",
  "gene": "UniProtKB:A0PJW8",
  "gene_symbol": "DAPL1",
  "term_id": "GO:0043022"
}